{
  "gene_name": "Methylthioribose-1-phosphate isomerase",
  "gene_symbol": "MRI1",
  "gene": "UniProtKB:Q9BV20",
  "term_id": "GO:0046523",
  "term_label": "S-methyl-5-thioribose-1-phosphate isomerase activity"
}